{
  "term_label": "Unknown molecular function",
  "gene_symbol": "WTAP",
  "gene": "UniProtKB:Q15007",
  "gene_name": "Pre-mRNA-splicing regulator WTAP",
  "term_id": "UNKNOWN:0001"
}